negative regulation of activin secretion [GO:0032336] (biological process) Definition: Any process that stops, prevents, or reduces the frequency, rate or extent of the regulated release of activin from a cell. Sources: GOC:mah Also known as: down regulation of activin secretion, down-regulation of activin secretion, downregulation of activin secretion, inhibition of activin secretion Relationships: is a type of regulation of activin secretion [GO:0032335]; is_a negative regulation of hormone secretion [GO:0046888]; negatively regulates GO:0032333